fertilization envelope [GO:0060387] (cellular component) Relationships: is_a egg coat [GO:0035805] Sources: GOC:dph, ISBN:0878932437 Also known as: fertilization membrane Definition: A structure that lies outside the plasma membrane and surrounds the egg. The fertilization envelope forms from the vitelline membrane after fertilization as a result of cortical granule release.